{
  "gene": "UniProtKB:Q86UP0",
  "term_label": "catenin complex",
  "gene_name": "Cadherin-24",
  "gene_symbol": "CDH24",
  "term_id": "GO:0016342"
}